{
  "term_label": "chromatin",
  "gene": "UniProtKB:O15178",
  "gene_symbol": "TBXT",
  "gene_name": "T-box transcription factor T",
  "term_id": "GO:0000785"
}